fatty acid beta-oxidation using acyl-CoA oxidase [GO:0033540] (BP) Sources: GOC:mah, MetaCyc:PWY-5136 Subtypes: GO:0140493 Relationships: is a type of fatty acid beta-oxidation [GO:0006635] Definition: A fatty acid beta-oxidation pathway in which the initial step, which converts an acyl-CoA to a trans-2-enoyl-CoA, is catalyzed by acyl-CoA oxidase; the electrons removed by oxidation pass directly to oxygen and produce hydrogen peroxide, which is cleaved by peroxisomal catalases. Fatty acid beta-oxidation begins with the addition of coenzyme A to a fatty acid, and ends when only two or three carbons remain (as acetyl-CoA or propionyl-CoA respectively).